metanephric nephron tubule morphogenesis [GO:0072282] (biological process) Definition: The process in which the anatomical structures of a metanephric nephron tubule are generated and organized. A metanephric nephron tubule is an epithelial tube that is part of the metanephric nephron, the functional part of the metanephros. Relationships: is a type of nephron tubule morphogenesis [GO:0072078]; is a type of metanephric tubule morphogenesis [GO:0072173]; is part of metanephric nephron tubule development [GO:0072234]; is part of GO:0072273 Sources: GOC:mtg_kidney_jan10 Subtypes: metanephric distal tubule morphogenesis [GO:0072287], metanephric proximal tubule morphogenesis [GO:0072288]